{
  "gene_symbol": "GRB14",
  "term_label": "insulin receptor signaling pathway",
  "term_id": "GO:0008286",
  "gene": "UniProtKB:Q14449",
  "gene_name": "Growth factor receptor-bound protein 14"
}